{
  "gene": "UniProtKB:Q8NH41",
  "gene_name": "Olfactory receptor 4K15",
  "term_id": "UNKNOWN:0002",
  "gene_symbol": "OR4K15",
  "term_label": "Unknown biological process"
}